{
  "gene": "UniProtKB:Q9H1R3",
  "gene_name": "Myosin light chain kinase 2, skeletal_cardiac muscle",
  "gene_symbol": "MYLK2",
  "term_label": "signal transduction",
  "term_id": "GO:0007165"
}